{
  "gene_name": "EF-hand calcium-binding domain-containing protein 7",
  "gene": "UniProtKB:A8K855",
  "term_id": "GO:1903569",
  "term_label": "positive regulation of protein localization to ciliary membrane",
  "gene_symbol": "EFCAB7"
}